respiratory burst [GO:0045730] (biological process) Regulation: regulated by regulation of respiratory burst [GO:0060263]; positively regulated by positive regulation of respiratory burst [GO:0060267]; negatively regulated by negative regulation of respiratory burst [GO:0060268] Subtypes: respiratory burst involved in defense response [GO:0002679], respiratory burst at fertilization [GO:0045729] Sources: ISBN:0198506732 Relationships: is a type of metabolic process [GO:0008152] Definition: A phase of elevated metabolic activity, during which oxygen consumption increases; this leads to the production, by an NADH dependent system, of hydrogen peroxide (H2O2), superoxide anions and hydroxyl radicals. Also known as: metabolic burst, oxidative burst